cardiac muscle cell apoptotic process [GO:0010659] (biological process) Regulation: regulated by GO:0010665; positively regulated by positive regulation of cardiac muscle cell apoptotic process [GO:0010666]; negatively regulated by negative regulation of cardiac muscle cell apoptotic process [GO:0010667] Sources: CL:0000746, GOC:dph, GOC:mtg_apoptosis, GOC:tb Also known as: cardiac muscle cell apoptosis Relationships: is a type of striated muscle cell apoptotic process [GO:0010658] Definition: A form of programmed cell death induced by external or internal signals that trigger the activity of proteolytic caspases, whose actions dismantle a cardiac muscle cell and result in its death. Cardiac muscle cells are striated muscle cells that are responsible for heart contraction.